{
  "term_id": "GO:0005635",
  "gene_name": "Importin-11",
  "gene_symbol": "IPO11",
  "term_label": "nuclear envelope",
  "gene": "UniProtKB:Q9UI26"
}